{
  "gene": "UniProtKB:P11226",
  "gene_name": "Mannose-binding protein C",
  "gene_symbol": "MBL2",
  "term_id": "GO:0005615",
  "term_label": "extracellular space"
}